{
  "gene": "UniProtKB:P35916",
  "gene_name": "Vascular endothelial growth factor receptor 3",
  "term_label": "cell migration",
  "term_id": "GO:0016477",
  "gene_symbol": "FLT4"
}